positive regulation of ceramide biosynthetic process [GO:2000304] (BP) Relationships: is a type of positive regulation of amide metabolic process [GO:0034250]; is a type of positive regulation of sphingolipid biosynthetic process [GO:0090154]; is_a regulation of ceramide biosynthetic process [GO:2000303]; positively regulates GO:0046513 Also known as: positive regulation of ceramide anabolism, positive regulation of ceramide biosynthesis, positive regulation of ceramide formation, positive regulation of ceramide synthesis Sources: GOC:dph Definition: Any process that activates or increases the frequency, rate or extent of ceramide biosynthetic process. Subtypes: positive regulation of glucosylceramide biosynthetic process [GO:0046319]